{
  "gene_name": "DNA-directed DNA_RNA polymerase mu",
  "gene": "UniProtKB:Q9NP87",
  "term_label": "nucleus",
  "gene_symbol": "POLM",
  "term_id": "GO:0005634"
}